{
  "term_id": "GO:0005025",
  "gene_name": "Serine_threonine-protein kinase receptor R3",
  "gene": "UniProtKB:P37023",
  "term_label": "transforming growth factor beta receptor activity, type I",
  "gene_symbol": "ACVRL1"
}